peripheral nervous system axon ensheathment [GO:0032292] (biological process) Relationships: is a type of GO:0008366 Also known as: ensheathment of axons in peripheral nervous system Sources: GOC:dgh Definition: The process in which a Schwann cell membrane closes around an axon in the peripheral nervous system. This can be a myelinating or a non-myelinating neuron-glial interaction. Subtypes: myelination in peripheral nervous system [GO:0022011], peripheral nervous system non-myelinated axon ensheathment [GO:0032294]